{
  "gene_symbol": "LETM1",
  "gene": "UniProtKB:O95202",
  "term_label": "mitochondrion",
  "term_id": "GO:0005739",
  "gene_name": "Mitochondrial proton_calcium exchanger protein"
}